{
  "gene_symbol": "CEBPA",
  "gene": "UniProtKB:P49715",
  "gene_name": "CCAAT_enhancer-binding protein alpha",
  "term_label": "DNA-binding transcription factor activity, RNA polymerase II-specific",
  "term_id": "GO:0000981"
}